{
  "gene": "UniProtKB:Q13003",
  "gene_name": "Glutamate receptor ionotropic, kainate 3",
  "term_label": "kainate selective glutamate receptor complex",
  "term_id": "GO:0032983",
  "gene_symbol": "GRIK3"
}